{
  "gene_name": "Protein lin-7 homolog C",
  "gene": "UniProtKB:Q9NUP9",
  "term_label": "synaptic vesicle transport",
  "term_id": "GO:0048489",
  "gene_symbol": "LIN7C"
}